{
  "gene": "UniProtKB:P10073",
  "term_label": "DNA-binding transcription factor activity, RNA polymerase II-specific",
  "gene_name": "Zinc finger and SCAN domain-containing protein 22",
  "term_id": "GO:0000981",
  "gene_symbol": "ZSCAN22"
}